nuclear matrix [GO:0016363] (cellular component) Definition: A dynamic, proteinaceous framework within the nucleus of eukaryotic cells, composed of proteins and RNA, that provides structural support for chromatin organization, gene regulation, and nuclear processes. References: PMID:15608168, PMID:3058729, PMID:39789220 Also known as: nucleoskeleton Relationships: is a type of cellular anatomical structure [GO:0110165]; is part of nuclear lumen [GO:0031981]